positive regulation of CD4-positive, alpha-beta T cell differentiation [GO:0043372] (biological process) Definition: Any process that activates or increases the frequency, rate or extent of CD4-positive, alpha-beta T cell differentiation. Sources: GOC:add, GOC:pr, ISBN:0781735149 Also known as: positive regulation of CD4-positive T lymphocyte differentiation, positive regulation of CD4-positive T-cell differentiation, positive regulation of CD4-positive T-lymphocyte differentiation, positive regulation of CD4-positive, alpha beta T cell differentiation, positive regulation of CD4-positive, alpha beta T lymphocyte differentiation, positive regulation of CD4-positive, alpha beta T-cell differentiation, positive regulation of CD4-positive, alpha beta T-lymphocyte differentiation, up regulation of CD4-positive, alpha beta T cell differentiation, up-regulation of CD4-positive, alpha beta T cell differentiation, upregulation of CD4-positive, alpha beta T cell differentiation, activation of CD4-positive, alpha beta T cell differentiation, stimulation of CD4-positive, alpha beta T cell differentiation, positive regulation of CD4-positive, alpha beta T cell development Note: Note that immunologists typically use the word 'development' to refer to cells of B or T cell lineages undergoing the process that GO describes as 'cell differentiation'. Relationships: is a type of GO:0043370; is_a positive regulation of alpha-beta T cell differentiation [GO:0046638]; is a type of GO:2000516; positively regulates CD4-positive, alpha-beta T cell differentiation [GO:0043367] Subtypes: positive regulation of CD4-positive, CD25-positive, alpha-beta regulatory T cell differentiation [GO:0032831], GO:0045624